{
  "gene_name": "UDP-glucuronosyltransferase 1-6",
  "term_id": "GO:0008210",
  "gene": "UniProtKB:P19224",
  "term_label": "estrogen metabolic process",
  "gene_symbol": "UGT1A6"
}